{
  "term_label": "Unknown molecular function",
  "gene_symbol": "PAG1",
  "gene_name": "Phosphoprotein associated with glycosphingolipid-enriched microdomains 1",
  "term_id": "UNKNOWN:0001",
  "gene": "UniProtKB:Q9NWQ8"
}